transport of virus in multicellular host [GO:0046739] (biological process) Relationships: is a type of GO:0044001; is a type of transport of virus [GO:0046794] Sources: GOC:bf, GOC:jl, ISBN:0781718325 Also known as: spread of virus within multicellular host, viral spread within multicellular host, spread of virus in multicellular host Subtypes: transport of virus in host, cell to cell [GO:0046740], transport of virus in host, tissue to tissue [GO:0046741] Definition: The transport of a virus between cells in a multicellular organism. The cells can be adjacent or spatially separated (e.g. in different tissues or organs).